{
  "gene_symbol": "SLC24A1",
  "gene": "UniProtKB:O60721",
  "term_id": "GO:0006874",
  "gene_name": "Sodium_potassium_calcium exchanger 1",
  "term_label": "intracellular calcium ion homeostasis"
}